{
  "gene_name": "Serine_threonine-protein kinase SMG1",
  "term_id": "GO:0005634",
  "term_label": "nucleus",
  "gene_symbol": "SMG1",
  "gene": "UniProtKB:Q96Q15"
}